initiation-specific glycolipid 1,6-alpha-mannosyltransferase activity [GO:0033164] (molecular function) Definition: Catalysis of the transfer of an alpha-D-mannosyl residue from GDP-mannose to Man(8)GlcNAc or Man(9)GlcNAc via an alpha-(1->6)-D-mannosyl-D-mannose linkage to form Man(9)GlcNAc or Man(10)GlcNAc, respectively. This is the first step specific to the biosynthesis of the outer chain of yeast mannoproteins. References: PMID:2644248 Sources: EC:2.4.1.232 Also known as: glycolipid 1,6-alpha-mannosyltransferase activity, glycolipid 6-alpha-mannosyltransferase activity, GDP-mannose:glycolipid 1,6-alpha-D-mannosyltransferase activity, GDP-mannose:oligosaccharide 1,6-alpha-D-mannosyltransferase activity, GDP-mannose:oligosaccharide 6-alpha-D-mannosyltransferase activity, initiation-specific alpha-1,6-mannosyltransferase activity Relationships: is_a alpha-1,6-mannosyltransferase activity [GO:0000009]